{
  "term_label": "regulation of lipid storage",
  "gene": "UniProtKB:P55055",
  "term_id": "GO:0010883",
  "gene_symbol": "NR1H2",
  "gene_name": "Oxysterols receptor LXR-beta"
}